membrane curvature sensor activity [GO:0140090] (molecular function) References: PMID:25898166 Relationships: is_a molecular sensor activity [GO:0140299]; has part lipid binding [GO:0008289] Definition: Preferential binding of proteins on curved membranes. The binding to curved membranes by insertion (aka wedging) to curved membranes is mediated by both the hydrophobic and hydrophilic faces of the helix of membrane curvature sensing (MCS) proteins.